{
  "gene_symbol": "CACNA1B",
  "gene_name": "Voltage-dependent N-type calcium channel subunit alpha-1B",
  "gene": "UniProtKB:Q00975",
  "term_id": "GO:0098703",
  "term_label": "calcium ion import across plasma membrane"
}